{
  "gene": "UniProtKB:Q14721",
  "term_id": "GO:0030424",
  "gene_symbol": "KCNB1",
  "term_label": "axon",
  "gene_name": "Potassium voltage-gated channel subfamily B member 1"
}